{
  "gene_name": "Uncharacterized protein C20orf144",
  "gene_symbol": "C20orf144",
  "term_label": "Unknown biological process",
  "term_id": "UNKNOWN:0002",
  "gene": "UniProtKB:Q9BQM9"
}